{
  "term_label": "catenin complex",
  "gene_name": "Cadherin-3",
  "gene": "UniProtKB:P22223",
  "gene_symbol": "CDH3",
  "term_id": "GO:0016342"
}